histone H3K4 monomethyltransferase activity [GO:0140945] (molecular function) Note: Comment: Note that the residue position corresponds to the canonical human H3 histone (UniProtKB:P84243); this residue is conserved across all eukaryotes. Residue 1 is the first residue following removal of the initiating Methionine (Met). Note that each histone is encoded by multiple genes, and sequences may vary across different genes within an organism. Relationships: is a type of histone H3K4 methyltransferase activity [GO:0042800] Definition: Catalysis of the reaction: L-lysyl4-[histone H3] + S-adenosyl-L-methionine = H+ + N6-methyl-L-lysyl4-[histone H3] + S-adenosyl-L-homocysteine. This reaction is the addition of a single methyl group to the unmethylated lysine residue at position 4 of histone H3, producing histone H3K4me. Also known as: histone H4-K4 methylation, histone H4K4 methylation, histone H3K4 monomethylase activity, histone lysine N-monomethyltransferase activity (H3-K4 specific) Sources: RHEA:60264